UDP-4-deoxy-4-formamido-beta-L-arabinopyranose biosynthetic process [GO:2001315] (BP) Sources: GOC:yaf, UniPathway:UPA00032 Definition: The chemical reactions and pathways resulting in the formation of a UDP-4-deoxy-4-formamido-beta-L-arabinopyranose. Relationships: is a type of nucleotide-sugar biosynthetic process [GO:0009226]; is a type of amino sugar biosynthetic process [GO:0046349] Also known as: UDP-4-deoxy-4-formamido-beta-L-arabinopyranose anabolism, UDP-4-deoxy-4-formamido-beta-L-arabinopyranose biosynthesis, UDP-4-deoxy-4-formamido-beta-L-arabinopyranose formation, UDP-4-deoxy-4-formamido-beta-L-arabinopyranose synthesis